high-affinity iron permease complex [GO:0033573] (cellular component) Also known as: high affinity iron permease complex References: PMID:16522632, PMID:8599111 Sources: GOC:jp Relationships: is a type of plasma membrane protein complex [GO:0098797]; is_a transmembrane transporter complex [GO:1902495]; is a type of ferroxidase complex [GO:1905862] Definition: A protein complex composed of a multicopper ferroxidase that oxidizes Fe(II) to Fe(III), and a ferric iron permease that transports the produced Fe(III) into the cell. In high-affinity transport the transporter is able to bind the solute even if it is only present at very low concentrations.